{
  "gene_name": "Lipid transferase CIDEB",
  "gene_symbol": "CIDEB",
  "term_id": "GO:0019915",
  "gene": "UniProtKB:Q9UHD4",
  "term_label": "lipid storage"
}